{
  "gene_symbol": "RMI2",
  "gene": "UniProtKB:Q96E14",
  "term_label": "regulation of sister chromatid segregation",
  "term_id": "GO:0033045",
  "gene_name": "RecQ-mediated genome instability protein 2"
}